{
  "gene_name": "Protein NYNRIN",
  "gene": "UniProtKB:Q9P2P1",
  "gene_symbol": "NYNRIN",
  "term_id": "GO:0003729",
  "term_label": "mRNA binding"
}